{
  "term_id": "UNKNOWN:0003",
  "gene": "UniProtKB:Q12894",
  "term_label": "Unknown cellular component",
  "gene_symbol": "IFRD2",
  "gene_name": "Interferon-related developmental regulator 2"
}